{
  "term_id": "GO:0019674",
  "gene_name": "Malate dehydrogenase, cytoplasmic",
  "gene_symbol": "MDH1",
  "term_label": "NAD+ metabolic process",
  "gene": "UniProtKB:P40925"
}